{
  "gene": "UniProtKB:P26367",
  "gene_name": "Paired box protein Pax-6",
  "term_id": "UNKNOWN:0003",
  "term_label": "Unknown cellular component",
  "gene_symbol": "PAX6"
}